{
  "gene": "UniProtKB:Q15386",
  "gene_symbol": "UBE3C",
  "term_id": "GO:0000209",
  "gene_name": "Ubiquitin-protein ligase E3C",
  "term_label": "protein polyubiquitination"
}